UDP-D-apiose biosynthetic process [GO:0033352] (biological process) Also known as: UDP-D-apiose anabolism, UDP-D-apiose biosynthesis, UDP-D-apiose formation, UDP-D-apiose synthesis Definition: The chemical reactions and pathways resulting in the formation of UDP-D-apiose, uridinediphosphoapicose, a substance composed of apiose in glycosidic linkage with uridine diphosphate. Relationships: is a type of nucleotide-sugar biosynthetic process [GO:0009226] Sources: GOC:mah, MetaCyc:PWY-5113